{
  "gene": "UniProtKB:Q16537",
  "gene_symbol": "PPP2R5E",
  "term_label": "protein phosphatase activator activity",
  "term_id": "GO:0072542",
  "gene_name": "Serine_threonine-protein phosphatase 2A 56 kDa regulatory subunit epsilon isoform"
}